{
  "term_label": "cytokine activity",
  "gene_name": "Transforming growth factor beta-1 proprotein",
  "gene": "UniProtKB:P01137",
  "term_id": "GO:0005125",
  "gene_symbol": "TGFB1"
}